regulation of interleukin-8 production [GO:0032677] (biological process) Subtypes: negative regulation of interleukin-8 production [GO:0032717], positive regulation of interleukin-8 production [GO:0032757] Relationships: is a type of regulation of cytokine production [GO:0001817]; regulates interleukin-8 production [GO:0032637] Also known as: regulation of IL-8 production, regulation of interleukin-8 biosynthetic process, regulation of interleukin-8 secretion Definition: Any process that modulates the frequency, rate, or extent of interleukin-8 production. Sources: GOC:mah